dermatan sulfate proteoglycan biosynthetic process [GO:0050651] (biological process) Definition: The chemical reactions and pathways resulting in the formation of dermatan sulfate proteoglycans, which consist of a core protein linked to a dermatan sulfate glycosaminoglycan. The dermatan sulfate chain is composed of the repeating disaccharide unit beta-(1,4)-D-hexuronic acid-beta-(1,3)-N-acetyl-D-galactosamine. Tthe former can be a mixture of sulfated and nonsulfated D-glucuronic and L-iduronic acids, and the latter can be O-sulfated. Dermatan sulfate chains are covalently linked to serine/threonine residues (O-linked) of the core protein via a tetrasaccharide linker sequence (xylose-galactose-galactose-glucuronate). References: PMID:17239763 Also known as: chondroitin sulfate B proteoglycan biosynthesis, chondroitin sulfate B proteoglycan biosynthetic process, dermatan sulfate proteoglycan anabolism, dermatan sulfate proteoglycan biosynthesis, dermatan sulfate proteoglycan formation, dermatan sulfate proteoglycan synthesis, dermatan sulphate proteoglycan biosynthesis, dermatan sulphate proteoglycan biosynthetic process Relationships: is a type of proteoglycan biosynthetic process [GO:0030166]; is a type of GO:0050655; is a type of protein O-linked glycosylation via xylose [GO:0180064]